pantetheine kinase activity [GO:0050165] (molecular function) Also known as: ATP:pantetheine 4'-phosphotransferase activity, pantetheine kinase (phosphorylating) Sources: EC:2.7.1.34, MetaCyc:PANTETHEINE-KINASE-RXN Relationships: is a type of kinase activity [GO:0016301]; is a type of GO:0016773 Definition: Catalysis of the reaction: ATP + pantetheine = ADP + pantetheine 4'-phosphate.